{
  "gene_symbol": "CD59",
  "term_label": "complement binding",
  "term_id": "GO:0001848",
  "gene": "UniProtKB:P13987",
  "gene_name": "CD59 glycoprotein"
}